mesonephric glomerular epithelial cell fate commitment [GO:0061252] (biological process) Subtypes: mesonephric glomerular parietal epithelial cell fate commitment [GO:0061255] Relationships: is a type of GO:0072314; is part of mesonephric glomerular epithelial cell differentiation [GO:0061250] Definition: The process in which the developmental fate of a cell becomes restricted such that it will develop into a mesonephric glomerular epithelial cell. Mesonephric glomerular epithelial cells are specialized epithelial cells that form part of the mesonephric glomerulus; there are two types, mesonephric glomerular parietal epithelial cells and mesonephric glomerular visceral epithelial cells. Sources: GOC:mtg_kidney_jan10